calcitriol binding [GO:1902098] (MF) Also known as: 1,25-dihydroxycholecalciferol binding, 1,25-dihydroxyvitamin D3 binding, 1alpha,25(OH)2 vitamin D3 binding, 1alpha,25(OH)2D3 binding, 1alpha,25-dihydroxycholecalciferol binding, 1alpha,25-dihydroxyvitamin D3 binding, hormonally active vitamin D3 binding Definition: Binding to calcitriol. Calcitriol (1,25-dihydroxycholecalciferol) is the hormonally active form of vitamin D3. References: PMID:21872797 Sources: GOC:TermGenie, Wikipedia:Calcitriol_receptor Relationships: is_a D3 vitamins binding [GO:1902271]